maintenance of protein location in mitochondrion [GO:0072656] (biological process) Definition: Any process in which a protein is maintained in a specific location in a mitochondrion, and is prevented from moving elsewhere. Sources: GOC:mah Relationships: is a type of maintenance of protein localization in organelle [GO:0072595]; is part of protein localization to mitochondrion [GO:0070585]; occurs in mitochondrion [GO:0005739]